{
  "gene": "UniProtKB:Q9Y3P8",
  "gene_symbol": "SIT1",
  "term_label": "plasma membrane",
  "gene_name": "Signaling threshold-regulating transmembrane adapter 1",
  "term_id": "GO:0005886"
}